{
  "term_id": "GO:0035332",
  "term_label": "positive regulation of hippo signaling",
  "gene_symbol": "FRMD1",
  "gene": "UniProtKB:Q8N878",
  "gene_name": "FERM domain-containing protein 1"
}